Roundabout signaling pathway [GO:0035385] (biological process) Also known as: ROBO signaling pathway, ROBO/SLIT signaling pathway, Roundabout signalling pathway Regulation: regulated by regulation of Roundabout signaling pathway [GO:0035386]; RO_0002212 by GO:0035387; positively regulated by positive regulation of Roundabout signaling pathway [GO:0035388] Definition: The series of molecular signals initiated by a SLIT protein binding to a Roundabout (ROBO) family receptor on the surface of a target cell, and ending with the regulation of a downstream cellular process, e.g. transcription. Sources: GOC:BHF, GOC:signaling Subtypes: Roundabout signaling pathway involved in axon guidance [GO:2001266], Roundabout signaling pathway involved in muscle cell chemotaxis toward tendon cell [GO:2001283] Relationships: is a type of cell surface receptor signaling pathway [GO:0007166]